{
  "gene_name": "Olfactory receptor family 1 subfamily R member 1 pseudogene",
  "term_id": "GO:0004984",
  "gene_symbol": "A0A286YEU6",
  "gene": "UniProtKB:A0A286YEU6",
  "term_label": "olfactory receptor activity"
}